regulation of cell cycle [GO:0051726] (biological process) Subtypes: GO:0007346, regulation of cell cycle process [GO:0010564], mitotic G2 cell cycle arrest in response to glucose starvation [GO:0036227], negative regulation of cell cycle [GO:0045786], positive regulation of cell cycle [GO:0045787], regulation of meiotic cell cycle [GO:0051445] Definition: Any process that modulates the rate or extent of progression through the cell cycle. Also known as: cell cycle modulation, cell cycle regulation, control of cell cycle progression, modulation of cell cycle progression, regulation of cell cycle progression, regulation of progression through cell cycle, arrest of mitotic cell cycle progression, cell cycle arrest, mitotic cell cycle arrest, negative regulation of cell cycle arrest, positive regulation of cell cycle arrest, regulation of cell cycle arrest, cell cycle regulator, tumor suppressor Relationships: is a type of GO:0050794; regulates cell cycle [GO:0007049] Sources: GOC:ai, GOC:dph, GOC:tb